{
  "gene": "UniProtKB:Q13625",
  "term_label": "nucleus",
  "term_id": "GO:0005634",
  "gene_name": "Apoptosis-stimulating of p53 protein 2",
  "gene_symbol": "TP53BP2"
}